{
  "term_id": "GO:0005667",
  "gene": "UniProtKB:Q8N196",
  "gene_name": "Homeobox protein SIX5",
  "term_label": "transcription regulator complex",
  "gene_symbol": "SIX5"
}